{
  "gene": "UniProtKB:Q13393",
  "term_id": "GO:0060627",
  "term_label": "regulation of vesicle-mediated transport",
  "gene_name": "Phospholipase D1",
  "gene_symbol": "PLD1"
}